hydrolase activity, acting on carbon-sulfur bonds [GO:0046508] (molecular function) Subtypes: adenosylhomocysteinase activity [GO:0004013], GO:0018740, UDPsulfoquinovose synthase activity [GO:0046507] Relationships: is a type of hydrolase activity [GO:0016787] Sources: GOC:jl Also known as: hydrolase activity, acting on carbon-sulphur bonds Definition: Catalysis of the hydrolysis of any carbon-sulfur bond, C-S.